regulation of TRAIL-activated apoptotic signaling pathway [GO:1903121] (biological process) Also known as: regulation of TRAIL-activated extrinsic apoptotic signaling pathway, regulation of TRAIL-induced apoptotic signaling pathway, regulation of tumor necrosis factor-related apoptosis-inducing ligand apoptotic signaling pathway Sources: GOC:PARL, GOC:TermGenie, GOC:bf, GO_REF:0000058 Subtypes: negative regulation of TRAIL-activated apoptotic signaling pathway [GO:1903122], positive regulation of TRAIL-activated apoptotic signaling pathway [GO:1903984] Relationships: is a type of GO:1902041; RO_0002211 GO:0036462 Definition: Any process that modulates the frequency, rate or extent of TRAIL-activated apoptotic signaling pathway.